{
  "term_label": "Unknown biological process",
  "gene": "UniProtKB:Q86UB2",
  "gene_symbol": "BIVM",
  "term_id": "UNKNOWN:0002",
  "gene_name": "Basic immunoglobulin-like variable motif-containing protein"
}